{
  "gene_symbol": "GNG11",
  "term_label": "heterotrimeric G-protein complex",
  "gene_name": "Guanine nucleotide-binding protein G(I)_G(S)_G(O) subunit gamma-11",
  "term_id": "GO:0005834",
  "gene": "UniProtKB:P61952"
}